{
  "term_label": "extracellular space",
  "term_id": "GO:0005615",
  "gene_symbol": "IL27",
  "gene": "UniProtKB:Q8NEV9",
  "gene_name": "Interleukin-27 subunit alpha"
}